{
  "gene_symbol": "ARHGEF26",
  "term_id": "UNKNOWN:0003",
  "term_label": "Unknown cellular component",
  "gene": "UniProtKB:Q96DR7",
  "gene_name": "Rho guanine nucleotide exchange factor 26"
}